endobrevin-SNAP-25-syntaxin-1a complex [GO:0070048] (cellular component) Definition: A SNARE complex that contains endobrevin (VAMP8), SNAP-25, and syntaxin 1a (or orthologs thereof). Also known as: SNARE complex (Stx1a, Snap25, Vamp8), Stx1a-Snap25-Vamp8 complex Relationships: is a type of SNARE complex [GO:0031201] References: PMID:10336434